response to selenite ion [GO:0072714] (biological process) Relationships: is a type of GO:1901700 Sources: GOC:mah Definition: Any process that results in a change in state or activity of a cell or an organism (in terms of movement, secretion, enzyme production, gene expression, etc.) as a result of a selenite ion stimulus. Subtypes: cellular response to selenite ion [GO:0072715]